{
  "gene": "UniProtKB:Q8IZF6",
  "gene_symbol": "ADGRG4",
  "term_id": "GO:0007186",
  "gene_name": "Adhesion G-protein coupled receptor G4",
  "term_label": "G protein-coupled receptor signaling pathway"
}